{
  "term_id": "GO:0005634",
  "gene_name": "PR domain zinc finger protein 14",
  "gene": "UniProtKB:Q9GZV8",
  "term_label": "nucleus",
  "gene_symbol": "PRDM14"
}